{
  "gene": "UniProtKB:O43916",
  "gene_name": "Carbohydrate sulfotransferase 1",
  "term_id": "GO:0006790",
  "term_label": "sulfur compound metabolic process",
  "gene_symbol": "CHST1"
}